{
  "gene_name": "ATPase family AAA domain-containing protein 2",
  "term_label": "nucleosome disassembly",
  "gene_symbol": "ATAD2",
  "gene": "UniProtKB:Q6PL18",
  "term_id": "GO:0006337"
}